postsynaptic neurotransmitter receptor activity [GO:0098960] (molecular function) Subtypes: dopamine neurotransmitter receptor activity [GO:0004952], GO:0015464, neurotransmitter receptor activity involved in regulation of postsynaptic membrane potential [GO:0099529], neurotransmitter receptor activity involved in regulation of postsynaptic cytosolic calcium ion concentration [GO:0099583] Definition: Neurotransmitter receptor activity occurring in the postsynaptic membrane during synaptic transmission. Sources: GOC:dos, GOC:signaling Also known as: neurotransmitter receptor activity involved in chemical synaptic transmission Relationships: is a type of neurotransmitter receptor activity [GO:0030594]; is part of chemical synaptic transmission, postsynaptic [GO:0099565]; BFO_0000066 postsynaptic membrane [GO:0045211]